{
  "term_id": "GO:0009311",
  "term_label": "oligosaccharide metabolic process",
  "gene_name": "Alpha-N-acetyl-neuraminyl-2,3-beta-galactosyl-1,3-N-acetyl-galactosaminide alpha-2,6-sialyltransferase",
  "gene": "UniProtKB:Q9H4F1",
  "gene_symbol": "ST6GALNAC4"
}